positive regulation of superoxide dismutase activity [GO:1901671] (biological process) Relationships: is a type of positive regulation of oxidoreductase activity [GO:0051353]; is a type of regulation of superoxide dismutase activity [GO:1901668]; positively regulates superoxide dismutase activity [GO:0004784] Definition: Any process that activates or increases the frequency, rate or extent of superoxide dismutase activity. Sources: GOC:TermGenie Also known as: activation of superoxide:superoxide oxidoreductase activity, positive regulation of superoxide:superoxide oxidoreductase activity, up regulation of superoxide dismutase activity, up regulation of superoxide:superoxide oxidoreductase activity, up-regulation of superoxide dismutase activity, up-regulation of superoxide:superoxide oxidoreductase activity, upregulation of superoxide dismutase activity, upregulation of superoxide:superoxide oxidoreductase activity, activation of Cu-Zn superoxide dismutase activity, activation of Mn, Fe superoxide dismutase, activation of copper, zinc superoxide dismutase activity, activation of ferrisuperoxide dismutase activity, activation of iron superoxide dismutase activity, activation of manganese superoxide dismutase activity, activation of nickel superoxide dismutase activity, activation of superoxide dismutase activity, positive regulation of Cu-Zn superoxide dismutase activity, positive regulation of Mn, Fe superoxide dismutase, positive regulation of copper, zinc superoxide dismutase activity, positive regulation of ferrisuperoxide dismutase activity, positive regulation of iron superoxide dismutase activity, positive regulation of manganese superoxide dismutase activity, positive regulation of nickel superoxide dismutase activity, up regulation of Cu-Zn superoxide dismutase activity, up regulation of Mn, Fe superoxide dismutase, up regulation of copper, zinc superoxide dismutase activity, up regulation of ferrisuperoxide dismutase activity, up regulation of iron superoxide dismutase activity, up regulation of manganese superoxide dismutase activity, up regulation of nickel superoxide dismutase activity, up-regulation of Cu-Zn superoxide dismutase activity, up-regulation of Mn, Fe superoxide dismutase, up-regulation of copper, zinc superoxide dismutase activity, up-regulation of ferrisuperoxide dismutase activity, up-regulation of iron superoxide dismutase activity, up-regulation of manganese superoxide dismutase activity, up-regulation of nickel superoxide dismutase activity, upregulation of Cu-Zn superoxide dismutase activity, upregulation of Mn, Fe superoxide dismutase, upregulation of copper, zinc superoxide dismutase activity, upregulation of ferrisuperoxide dismutase activity, upregulation of iron superoxide dismutase activity, upregulation of manganese superoxide dismutase activity, upregulation of nickel superoxide dismutase activity, activation of Cu,Zn-SOD, activation of Fe-SOD, activation of Mn-SOD, activation of SOD, activation of SOD-1, activation of SOD-2, activation of SOD-3, activation of SOD-4, activation of SODF, activation of SODS, activation of cuprein, activation of cytocuprein, activation of erythrocuprein, activation of hemocuprein, activation of hepatocuprein, activation of iron superoxide oxidoreductase, activation of manganese superoxide oxidoreductase, activation of nickel superoxide oxidoreductase, activation of superoxide dismutase I, activation of superoxide dismutase II, activation of zinc superoxide oxidoreductase, positive regulation of Cu,Zn-SOD, positive regulation of Fe-SOD, positive regulation of Mn-SOD, positive regulation of SOD, positive regulation of SOD-1, positive regulation of SOD-2, positive regulation of SOD-3, positive regulation of SOD-4, positive regulation of SODF, positive regulation of SODS, positive regulation of cuprein, positive regulation of cytocuprein, positive regulation of erythrocuprein, positive regulation of hemocuprein, positive regulation of hepatocuprein, positive regulation of iron superoxide oxidoreductase, positive regulation of manganese superoxide oxidoreductase, positive regulation of nickel superoxide oxidoreductase, positive regulation of superoxide dismutase I, positive regulation of superoxide dismutase II, positive regulation of zinc superoxide oxidoreductase, up regulation of Cu,Zn-SOD, up regulation of Fe-SOD, up regulation of Mn-SOD, up regulation of SOD, up regulation of SOD-1, up regulation of SOD-2, up regulation of SOD-3, up regulation of SOD-4, up regulation of SODF, up regulation of SODS, up regulation of cuprein, up regulation of cytocuprein, up regulation of erythrocuprein, up regulation of hemocuprein, up regulation of hepatocuprein, up regulation of iron superoxide oxidoreductase, up regulation of manganese superoxide oxidoreductase, up regulation of nickel superoxide oxidoreductase, up regulation of superoxide dismutase I, up regulation of superoxide dismutase II, up regulation of zinc superoxide oxidoreductase, up-regulation of Cu,Zn-SOD, up-regulation of Fe-SOD, up-regulation of Mn-SOD, up-regulation of SOD, up-regulation of SOD-1, up-regulation of SOD-2, up-regulation of SOD-3, up-regulation of SOD-4, up-regulation of SODF, up-regulation of SODS, up-regulation of cuprein, up-regulation of cytocuprein, up-regulation of erythrocuprein, up-regulation of hemocuprein, up-regulation of hepatocuprein, up-regulation of iron superoxide oxidoreductase, up-regulation of manganese superoxide oxidoreductase, up-regulation of nickel superoxide oxidoreductase, up-regulation of superoxide dismutase I, up-regulation of superoxide dismutase II, up-regulation of zinc superoxide oxidoreductase, upregulation of Cu,Zn-SOD, upregulation of Fe-SOD, upregulation of Mn-SOD, upregulation of SOD, upregulation of SOD-1, upregulation of SOD-2, upregulation of SOD-3, upregulation of SOD-4, upregulation of SODF, upregulation of SODS, upregulation of cuprein, upregulation of cytocuprein, upregulation of erythrocuprein, upregulation of hemocuprein, upregulation of hepatocuprein, upregulation of iron superoxide oxidoreductase, upregulation of manganese superoxide oxidoreductase, upregulation of nickel superoxide oxidoreductase, upregulation of superoxide dismutase I, upregulation of superoxide dismutase II, upregulation of zinc superoxide oxidoreductase